{
  "term_id": "UNKNOWN:0002",
  "gene_symbol": "SBSPON",
  "gene": "UniProtKB:Q8IVN8",
  "term_label": "Unknown biological process",
  "gene_name": "Somatomedin-B and thrombospondin type-1 domain-containing protein"
}